{
  "term_id": "GO:0043005",
  "gene_symbol": "CAMK2B",
  "gene": "UniProtKB:Q13554",
  "gene_name": "Calcium_calmodulin-dependent protein kinase type II subunit beta",
  "term_label": "neuron projection"
}